{
  "term_label": "Unknown cellular component",
  "gene_symbol": "CBLL2",
  "gene": "UniProtKB:Q8N7E2",
  "gene_name": "E3 ubiquitin-protein ligase CBLL2",
  "term_id": "UNKNOWN:0003"
}